transporter inhibitor activity [GO:0141110] (molecular function) Relationships: is a type of GO:0140678; is a type of transporter regulator activity [GO:0141108]; negatively regulates GO:0005215 Definition: Binds to and stops, prevents, or reduces the activity of a transporter. Subtypes: channel inhibitor activity [GO:0016248], GO:0097690 Sources: GOC:curators